{
  "gene_symbol": "DET1",
  "gene": "UniProtKB:Q7L5Y6",
  "term_id": "GO:0031461",
  "gene_name": "DET1 homolog",
  "term_label": "cullin-RING ubiquitin ligase complex"
}